{
  "term_label": "microtubule binding",
  "gene": "UniProtKB:Q9Y496",
  "gene_symbol": "KIF3A",
  "term_id": "GO:0008017",
  "gene_name": "Kinesin-like protein KIF3A"
}